{
  "term_id": "UNKNOWN:0003",
  "term_label": "Unknown cellular component",
  "gene": "UniProtKB:Q8IZP1",
  "gene_symbol": "TBC1D3",
  "gene_name": "TBC1 domain family member 3"
}